{
  "gene_name": "FYVE, RhoGEF and PH domain-containing protein 3",
  "gene": "UniProtKB:Q5JSP0",
  "term_label": "filopodium assembly",
  "term_id": "GO:0046847",
  "gene_symbol": "FGD3"
}